NoRC complex [GO:0090536] (cellular component) Relationships: is a type of ISWI-type complex [GO:0031010] Sources: GOC:krc Definition: An ISWI complex that contains an ATPase subunit of the ISWI family (specifically SNF2H in mammals, which contain two ISWI homologs) and a Tip5 homolog. In mammals, NoRC is involved in regulation of transcription from RNAP I and RNA polymerase III promoters.